histone pre-mRNA DCP binding [GO:0071208] (molecular function) References: PMID:19470752 Relationships: is a type of GO:0003723 Definition: Binding to the downstream cleavage product (DCP) generated by histone pre-mRNA 3'-end processing.